{
  "term_id": "GO:0009897",
  "gene_symbol": "TFRC",
  "term_label": "external side of plasma membrane",
  "gene": "UniProtKB:P02786",
  "gene_name": "Transferrin receptor protein 1"
}